ribosome localization [GO:0033750] (biological process) Subtypes: GO:0000054 Definition: A process in which a ribosome is transported to, and/or maintained in, a specific location. Also known as: establishment of ribosome localisation, establishment of ribosome localization, ribosome localisation Sources: GOC:mah Relationships: is_a organelle localization [GO:0051640]